negative regulation of anterograde axonal transport of mitochondrion [GO:0061882] (biological process) Also known as: negative regulation of anterograde axon transport of mitochondria Relationships: is a type of negative regulation of intracellular transport [GO:0032387]; is a type of regulation of anterograde axonal transport of mitochondrion [GO:0061880]; negatively regulates anterograde axonal transport of mitochondrion [GO:0098957] References: PMID:24302729 Definition: Any process that stops, prevents, or reduces the frequency, rate or extent of the directed movement of mitochondria along microtubules in axons away from the cell body and towards the presynapse.